regulation of gap junction assembly [GO:1903596] (biological process) References: PMID:25017399 Sources: GOC:BHF, GOC:TermGenie, GOC:mtg_cardiac_conduct_nov11, GOC:rl, GO_REF:0000058 Subtypes: negative regulation of gap junction assembly [GO:1903597], GO:1903598 Relationships: is a type of GO:1901888; regulates GO:0016264 Definition: Any process that modulates the frequency, rate or extent of gap junction assembly.